protein histidine kinase activity [GO:0004673] (molecular function) Relationships: is a type of protein kinase activity [GO:0004672]; is a type of phosphotransferase activity, nitrogenous group as acceptor [GO:0016775]; BFO_0000050 peptidyl-histidine phosphorylation [GO:0018106] Subtypes: phosphorelay sensor kinase activity [GO:0000155], protein histidine pros-kinase activity [GO:0008256], protein histidine tele-kinase activity [GO:0008257], transmembrane receptor histidine kinase activity [GO:0009784] Also known as: histidine kinase activity, protein-histidine kinase activity, ATP:protein-L-histidine N-phosphotransferase activity, histidine protein kinase activity, protein kinase (histidine) Definition: Catalysis of the reaction: ATP + protein L-histidine = ADP + protein phospho-L-histidine. Sources: EC:2.7.13.3, GOC:mah